{
  "gene": "UniProtKB:Q4KMZ1",
  "term_label": "Unknown cellular component",
  "term_id": "UNKNOWN:0003",
  "gene_symbol": "IQCC",
  "gene_name": "IQ domain-containing protein C"
}